{
  "gene_name": "Ankyrin repeat domain-containing protein 26",
  "term_label": "Unknown molecular function",
  "gene_symbol": "ANKRD26",
  "gene": "UniProtKB:Q9UPS8",
  "term_id": "UNKNOWN:0001"
}